{
  "gene_name": "Neuroblast differentiation-associated protein AHNAK",
  "gene_symbol": "AHNAK",
  "gene": "UniProtKB:Q09666",
  "term_id": "GO:0043484",
  "term_label": "regulation of RNA splicing"
}